{
  "gene": "UniProtKB:O15397",
  "term_id": "GO:0006606",
  "gene_name": "Importin-8",
  "gene_symbol": "IPO8",
  "term_label": "protein import into nucleus"
}